perforant pathway to dendrate granule cell synapse [GO:0140240] (cellular component) Also known as: perforant pathway to DG granule cell synapse Relationships: is a type of synapse [GO:0045202] Definition: A neuron to neuron synapse of a pyramidal neuron in the entorhinal cortex onto a granule cell in the dentate gyrus of the hippocampus. References: PMID:22727665, PMID:29199135